integrin alpha1-beta1 complex [GO:0034665] (cellular component) References: PMID:12297042 Also known as: VLA-1 complex, alpha1-beta1 integrin complex, ITGA1-ITGB1 complex Relationships: is a type of integrin complex [GO:0008305] Definition: An integrin complex that comprises one alpha1 subunit and one beta1 subunit.